(-)-secoisolariciresinol catabolic process [GO:1902137] (biological process) Definition: The chemical reactions and pathways resulting in the breakdown of (-)-secoisolariciresinol. Relationships: is a type of phenol-containing compound catabolic process [GO:0019336]; is a type of GO:0034313; is a type of lignan catabolic process [GO:0046273] Also known as: (-)-secoisolariciresinol breakdown, (-)-secoisolariciresinol catabolism, (-)-secoisolariciresinol degradation References: PMID:8910615, PMID:9872995 Sources: GOC:TermGenie